{
  "term_id": "GO:0006081",
  "gene_symbol": "ALDH1A2",
  "gene": "UniProtKB:O94788",
  "gene_name": "Retinal dehydrogenase 2",
  "term_label": "aldehyde metabolic process"
}